response to transforming growth factor beta [GO:0071559] (biological process) Subtypes: cellular response to transforming growth factor beta stimulus [GO:0071560] Relationships: is a type of response to growth factor [GO:0070848] Sources: GOC:mah Also known as: response to TGF-beta stimulus, response to TGFbeta stimulus, response to transforming growth factor beta stimulus Definition: Any process that results in a change in state or activity of a cell or an organism (in terms of movement, secretion, enzyme production, gene expression, etc.) as a result of a transforming growth factor beta stimulus.